L-galactose dehydrogenase activity [GO:0010349] (molecular function) Definition: Catalysis of the reaction: L-galactose + NAD+ = L-galactono-1,4-lactone + NADH + H+. References: PMID:12047629 Sources: RHEA:31559 Also known as: L-galactose 1-dehydrogenase activity Relationships: is_a GO:0016616